{
  "term_label": "Unknown molecular function",
  "gene_symbol": "Q8N377",
  "gene": "UniProtKB:Q8N377",
  "gene_name": "Putative uncharacterized protein LOC387726",
  "term_id": "UNKNOWN:0001"
}